flower development [GO:0009908] (biological process) Definition: The process whose specific outcome is the progression of the flower over time, from its formation to the mature structure. The flower is the reproductive structure in a plant, and its development begins with the transition of the vegetative or inflorescence meristem into a floral meristem. Sources: GOC:tb, ISBN:0879015322 Relationships: is a type of reproductive shoot system development [GO:0090567] Regulation: regulated by regulation of flower development [GO:0009909]; negatively regulated by GO:0009910; positively regulated by positive regulation of flower development [GO:0009911]